{
  "term_label": "MAP kinase kinase activity",
  "gene": "UniProtKB:P36507",
  "term_id": "GO:0004708",
  "gene_symbol": "MAP2K2",
  "gene_name": "Dual specificity mitogen-activated protein kinase kinase 2"
}